{
  "gene": "UniProtKB:Q96K31",
  "term_label": "Unknown cellular component",
  "gene_name": "Uncharacterized protein C8orf76",
  "gene_symbol": "C8orf76",
  "term_id": "UNKNOWN:0003"
}